protein K63-linked ubiquitination [GO:0070534] (biological process) References: PMID:15556404 Sources: GOC:mah Definition: A protein ubiquitination process in which a polymer of ubiquitin, formed by linkages between lysine residues at position 63 of the ubiquitin monomers, is added to a protein. K63-linked ubiquitination does not target the substrate protein for degradation, but is involved in several pathways, notably as a signal to promote error-free DNA postreplication repair. Relationships: is a type of protein polyubiquitination [GO:0000209] Regulation: regulated by regulation of protein K63-linked ubiquitination [GO:1900044]; negatively regulated by negative regulation of protein K63-linked ubiquitination [GO:1900045]; positively regulated by positive regulation of protein K63-linked ubiquitination [GO:1902523] Also known as: protein K63-linked polyubiquitination